chondroitin-sulfate-ABC exolyase activity [GO:0034001] (molecular function) Definition: Catalysis of the exolytic cleavage of disaccharide residues from the non-reducing ends of both polymeric chondroitin sulfates and their oligosaccharide fragments. Sources: EC:4.2.2.21 Also known as: ChS ABC lyase activity, chondroitin ABC eliminase activity, chondroitin sulfate ABC lyase activity, chondroitinase ABC activity, chondroitinase activity, ChS ABC lyase II activity, chondroitin sulfate ABC exoeliminase activity, chondroitin sulfate ABC exolyase activity Relationships: is a type of carbon-oxygen lyase activity, acting on polysaccharides [GO:0016837]